{
  "gene_name": "Ataxin-3",
  "gene": "UniProtKB:P54252",
  "term_label": "positive regulation of ERAD pathway",
  "term_id": "GO:1904294",
  "gene_symbol": "ATXN3"
}